{
  "gene": "UniProtKB:Q08174",
  "gene_name": "Protocadherin-1",
  "term_id": "GO:0005886",
  "gene_symbol": "PCDH1",
  "term_label": "plasma membrane"
}